{
  "gene_symbol": "LINC01547",
  "term_id": "UNKNOWN:0002",
  "term_label": "Unknown biological process",
  "gene": "UniProtKB:P58512",
  "gene_name": "Uncharacterized protein encoded by LINC01547"
}